{
  "term_id": "GO:0007015",
  "gene_name": "Protein POF1B",
  "term_label": "actin filament organization",
  "gene_symbol": "POF1B",
  "gene": "UniProtKB:Q8WVV4"
}